{
  "term_label": "Unknown biological process",
  "gene_symbol": "DLK2",
  "gene": "UniProtKB:Q6UY11",
  "term_id": "UNKNOWN:0002",
  "gene_name": "Protein delta homolog 2"
}